oenocyte differentiation [GO:0001742] (biological process) Sources: GOC:go_curators Also known as: oenocyte cell differentiation Relationships: is a type of cell differentiation [GO:0030154] Definition: The process in which a relatively unspecialized cell acquires the specialized features of an oenocyte. Oenocytes are large secretory cells found in clusters underlying the epidermis of larval abdominal segments.